{
  "term_id": "GO:0008083",
  "term_label": "growth factor activity",
  "gene": "UniProtKB:Q9NP95",
  "gene_symbol": "FGF20",
  "gene_name": "Fibroblast growth factor 20"
}